{
  "term_id": "GO:0005737",
  "gene_name": "Developmentally-regulated GTP-binding protein 2",
  "gene": "UniProtKB:P55039",
  "gene_symbol": "DRG2",
  "term_label": "cytoplasm"
}